nephron tubule development [GO:0072080] (biological process) Sources: GOC:mtg_kidney_jan10 Definition: The progression of a nephron tubule over time, from its initial formation to the mature structure. A nephron tubule is an epithelial tube that is part of the nephron, the functional part of the kidney. Subtypes: pronephric nephron tubule development [GO:0039020], mesonephric nephron tubule development [GO:0061242], proximal tubule development [GO:0072014], distal tubule development [GO:0072017], GO:0072019, proximal straight tubule development [GO:0072020], ascending thin limb development [GO:0072021], thick ascending limb development [GO:0072023], distal convoluted tubule development [GO:0072025], connecting tubule development [GO:0072027], loop of Henle development [GO:0072070], GO:0072234 Relationships: is a type of GO:0061326; is a type of nephron epithelium development [GO:0072009]